positive regulation of oxidative phosphorylation uncoupler activity [GO:2000277] (biological process) Sources: GOC:mah Definition: Any process that activates or increases the frequency, rate or extent of oxidative phosphorylation uncoupler activity. Also known as: positive regulation of mitochondrial uncoupling protein activity, positive regulation of uncoupling protein activity Relationships: is a type of GO:0022898; is a type of positive regulation of transporter activity [GO:0032411]; positively regulates oxidative phosphorylation uncoupler activity [GO:0017077]